{
  "gene_name": "Small integral membrane protein 17",
  "gene_symbol": "SMIM17",
  "term_label": "Unknown cellular component",
  "gene": "UniProtKB:P0DL12",
  "term_id": "UNKNOWN:0003"
}